{
  "gene_name": "Amphoterin-induced protein 1",
  "term_label": "membrane",
  "gene_symbol": "AMIGO1",
  "term_id": "GO:0016020",
  "gene": "UniProtKB:Q86WK6"
}